positive regulation of reticulophagy [GO:0140501] (biological process) Relationships: is a type of positive regulation of macroautophagy [GO:0016239]; is a type of regulation of reticulophagy [GO:0140500]; positively regulates reticulophagy [GO:0061709] References: PMID:32735772 Definition: Any process that increases the frequency, rate or extent of reticulophagy. Also known as: positive regulation of ER autophagy, positive regulation of ER-phagy, positive regulation of autophagy of the ER, positive regulation of autophagy of the endoplasmic reticulum, positive regulation of endoplasmic reticulum autophagy, positive regulation of ER degradation, positive regulation of endoplasmic reticulum degradation